{
  "gene": "UniProtKB:Q9BXW4",
  "gene_name": "Microtubule-associated proteins 1A_1B light chain 3C",
  "term_label": "mitophagy",
  "gene_symbol": "MAP1LC3C",
  "term_id": "GO:0000423"
}